{
  "gene": "UniProtKB:Q9BXX3",
  "gene_name": "Ankyrin repeat domain-containing protein 30A",
  "term_label": "Unknown molecular function",
  "term_id": "UNKNOWN:0001",
  "gene_symbol": "ANKRD30A"
}